{
  "term_id": "GO:0001228",
  "gene": "UniProtKB:Q86UD4",
  "term_label": "DNA-binding transcription activator activity, RNA polymerase II-specific",
  "gene_symbol": "ZNF329",
  "gene_name": "Zinc finger protein 329"
}